{
  "term_label": "regulation of DNA-templated transcription",
  "term_id": "GO:0006355",
  "gene": "UniProtKB:Q8TF32",
  "gene_symbol": "ZNF431",
  "gene_name": "Zinc finger protein 431"
}